{
  "term_id": "GO:0003724",
  "gene_name": "Probable ATP-dependent RNA helicase DDX20",
  "gene_symbol": "DDX20",
  "gene": "UniProtKB:Q9UHI6",
  "term_label": "RNA helicase activity"
}